{
  "term_label": "Unknown molecular function",
  "gene_symbol": "C5orf24",
  "term_id": "UNKNOWN:0001",
  "gene_name": "UPF0461 protein C5orf24",
  "gene": "UniProtKB:Q7Z6I8"
}